assembly of apicomedial cortex actomyosin [GO:0106036] (biological process) Definition: A process which results in the assembly or arrangement of constituent parts apicomedial cortex actomyosin. Relationships: is a type of cortical actin cytoskeleton organization [GO:0030866]; is a type of actomyosin structure organization [GO:0031032] References: PMID:28263180